{
  "term_label": "ceramide biosynthetic process",
  "term_id": "GO:0046513",
  "gene": "UniProtKB:Q71RH2",
  "gene_symbol": "TLCD3B",
  "gene_name": "Ceramide synthase"
}